{
  "term_label": "intracellular calcium ion homeostasis",
  "gene_symbol": "ATP13A3",
  "gene": "UniProtKB:Q9H7F0",
  "gene_name": "Polyamine-transporting ATPase 13A3",
  "term_id": "GO:0006874"
}